{
  "term_label": "Unknown cellular component",
  "gene_symbol": "SPDYE1",
  "gene_name": "Speedy protein E1",
  "term_id": "UNKNOWN:0003",
  "gene": "UniProtKB:Q8NFV5"
}